{
  "term_id": "GO:0004888",
  "gene_symbol": "LAIR2",
  "gene_name": "Leukocyte-associated immunoglobulin-like receptor 2",
  "term_label": "transmembrane signaling receptor activity",
  "gene": "UniProtKB:Q6ISS4"
}